glycerone kinase activity [GO:0004371] (molecular function) Sources: EC:2.7.1.29, RHEA:15773 Definition: Catalysis of the reaction: ATP + glycerone = ADP + glycerone phosphate + 2 H+. Relationships: is a type of GO:0016301; is a type of phosphotransferase activity, alcohol group as acceptor [GO:0016773] Also known as: ATP:glycerone phosphotransferase activity, acetol kinase (phosphorylating), acetol kinase activity, dihydroxyacetone kinase activity